{
  "term_id": "UNKNOWN:0002",
  "gene_name": "Uncharacterized protein",
  "term_label": "Unknown biological process",
  "gene_symbol": "A0A0G2JND7",
  "gene": "UniProtKB:A0A0G2JND7"
}